{
  "gene": "UniProtKB:Q99811",
  "gene_name": "Paired mesoderm homeobox protein 2",
  "gene_symbol": "PRRX2",
  "term_label": "regulation of transcription by RNA polymerase II",
  "term_id": "GO:0006357"
}